{
  "gene": "UniProtKB:Q8N5Y8",
  "term_label": "protein serine/threonine kinase activator activity",
  "term_id": "GO:0043539",
  "gene_name": "Protein mono-ADP-ribosyltransferase PARP16",
  "gene_symbol": "PARP16"
}